{
  "gene_name": "UPF0488 protein C8orf33",
  "gene_symbol": "C8orf33",
  "gene": "UniProtKB:Q9H7E9",
  "term_label": "Unknown cellular component",
  "term_id": "UNKNOWN:0003"
}